response to xylene [GO:1901501] (biological process) Sources: GOC:TermGenie, GOC:mengo_curators Relationships: is_a GO:0042221 Subtypes: response to p-xylene [GO:1901500] Definition: Any process that results in a change in state or activity of a cell or an organism (in terms of movement, secretion, enzyme production, gene expression, etc.) as a result of a xylene stimulus.